{
  "gene": "UniProtKB:Q70E73",
  "gene_symbol": "RAPH1",
  "gene_name": "Ras-associated and pleckstrin homology domains-containing protein 1",
  "term_id": "GO:0030674",
  "term_label": "protein-macromolecule adaptor activity"
}